{
  "gene_name": "Protein XRP2",
  "term_label": "post-Golgi vesicle-mediated transport",
  "term_id": "GO:0006892",
  "gene": "UniProtKB:O75695",
  "gene_symbol": "RP2"
}